{
  "gene_symbol": "TRIP13",
  "gene_name": "Pachytene checkpoint protein 2 homolog",
  "gene": "UniProtKB:Q15645",
  "term_label": "meiotic recombination checkpoint signaling",
  "term_id": "GO:0051598"
}